{
  "term_id": "GO:0048666",
  "gene_name": "Rhox homeobox family member 1",
  "term_label": "neuron development",
  "gene": "UniProtKB:Q8NHV9",
  "gene_symbol": "RHOXF1"
}